{
  "gene_name": "Regulatory-associated protein of mTOR",
  "term_label": "cellular response to starvation",
  "gene_symbol": "RPTOR",
  "term_id": "GO:0009267",
  "gene": "UniProtKB:Q8N122"
}